{
  "term_label": "apical plasma membrane",
  "gene_symbol": "SLC34A3",
  "gene_name": "Sodium-dependent phosphate transport protein 2C",
  "term_id": "GO:0016324",
  "gene": "UniProtKB:Q8N130"
}